{
  "term_id": "GO:0005125",
  "gene_name": "Growth_differentiation factor 8",
  "term_label": "cytokine activity",
  "gene": "UniProtKB:O14793",
  "gene_symbol": "MSTN"
}